dipeptide transmembrane transport [GO:0035442] (biological process) Also known as: dipeptide membrane transport Relationships: is a type of oligopeptide transmembrane transport [GO:0035672]; is a type of dipeptide transport [GO:0042938] Sources: GOC:vw Note: Note that this term is not intended for use in annotating lateral movement within membranes. Definition: The directed movement of a dipeptide across a membrane by means of some agent such as a transporter or pore. A dipeptide is a combination of two amino acids linked together by a peptide (-CO-NH-) bond. Subtypes: GO:0140206, p-aminobenzoyl-glutamate transmembrane transport [GO:1902604] Regulation: RO_0002211 by regulation of dipeptide transmembrane transport [GO:2001148]; negatively regulated by negative regulation of dipeptide transmembrane transport [GO:2001149]; positively regulated by positive regulation of dipeptide transmembrane transport [GO:2001150]